{
  "term_label": "skeletal system development",
  "gene": "UniProtKB:Q9GZV7",
  "gene_name": "Hyaluronan and proteoglycan link protein 2",
  "term_id": "GO:0001501",
  "gene_symbol": "HAPLN2"
}